{
  "gene_symbol": "H2BC1",
  "term_id": "GO:0006325",
  "term_label": "chromatin organization",
  "gene_name": "Histone H2B type 1-A",
  "gene": "UniProtKB:Q96A08"
}